{
  "term_id": "UNKNOWN:0001",
  "gene_symbol": "ELMOD3",
  "term_label": "Unknown molecular function",
  "gene": "UniProtKB:Q96FG2",
  "gene_name": "ELMO domain-containing protein 3"
}